{
  "gene_symbol": "MYSM1",
  "term_id": "GO:0006338",
  "term_label": "chromatin remodeling",
  "gene_name": "Deubiquitinase MYSM1",
  "gene": "UniProtKB:Q5VVJ2"
}